{
  "term_label": "DNA-binding transcription factor activity, RNA polymerase II-specific",
  "gene_name": "T-box transcription factor TBX18",
  "gene_symbol": "TBX18",
  "gene": "UniProtKB:O95935",
  "term_id": "GO:0000981"
}